{
  "gene": "UniProtKB:Q8N9I0",
  "term_id": "GO:0005544",
  "term_label": "calcium-dependent phospholipid binding",
  "gene_name": "Synaptotagmin-2",
  "gene_symbol": "SYT2"
}